bacteroid-containing symbiosome [GO:0043660] (cellular component) Subtypes: organellar chromatophore [GO:0070111] Sources: GOC:cc Definition: A symbiosome containing any of various structurally modified bacteria, such as those occurring on the root nodules of leguminous plants. Relationships: is a type of symbiosome [GO:0043659]